{
  "term_label": "Unknown biological process",
  "gene_name": "UDP-N-acetylglucosamine--dolichyl-phosphate N-acetylglucosaminephosphotransferase",
  "gene": "UniProtKB:Q9H3H5",
  "term_id": "UNKNOWN:0002",
  "gene_symbol": "DPAGT1"
}